{
  "term_label": "regulation of lysosomal membrane permeability",
  "gene_symbol": "LAPTM5",
  "gene_name": "Lysosomal-associated transmembrane protein 5",
  "term_id": "GO:0097213",
  "gene": "UniProtKB:Q13571"
}